{
  "gene": "UniProtKB:A6NP11",
  "gene_name": "Zinc finger protein 716",
  "term_label": "regulation of DNA-templated transcription",
  "term_id": "GO:0006355",
  "gene_symbol": "ZNF716"
}